regulation of satellite cell activation involved in skeletal muscle regeneration [GO:0014717] (biological process) Definition: Any process that modulates the frequency, rate or extent of satellite cell activation. The satellite cell activation is the process that initiates satellite cell division by causing it to move from quiescence to the G1 stage of the cell cycle. The cell swells and there are a number of other small changes. The cells then start to divide. Following cell division the cells will differentiate. Relationships: is a type of regulation of skeletal muscle tissue regeneration [GO:0043416]; is a type of GO:0050865; regulates satellite cell activation involved in skeletal muscle regeneration [GO:0014901] Sources: GOC:mtg_muscle Subtypes: positive regulation of satellite cell activation involved in skeletal muscle regeneration [GO:0014718], GO:1901667